{
  "term_id": "GO:0005525",
  "gene": "UniProtKB:Q9BUF5",
  "gene_symbol": "TUBB6",
  "gene_name": "Tubulin beta-6 chain",
  "term_label": "GTP binding"
}